{
  "gene_symbol": "RGL3",
  "gene_name": "Ral guanine nucleotide dissociation stimulator-like 3",
  "gene": "UniProtKB:Q3MIN7",
  "term_label": "plasma membrane",
  "term_id": "GO:0005886"
}